{
  "term_id": "GO:0043651",
  "gene": "UniProtKB:O75342",
  "gene_name": "Arachidonate 12-lipoxygenase, 12R-type",
  "gene_symbol": "ALOX12B",
  "term_label": "linoleic acid metabolic process"
}